positive regulation of uterine smooth muscle contraction [GO:0070474] (biological process) Also known as: positive regulation of myometrial contraction, positive regulation of myometrial smooth muscle contraction, positive regulation of myometrium contraction, up regulation of uterine smooth muscle contraction, up-regulation of uterine smooth muscle contraction, upregulation of uterine smooth muscle contraction, activation of uterine smooth muscle contraction, stimulation of uterine smooth muscle contraction Definition: Any process that increases the frequency, rate or extent of uterine smooth muscle contraction. Relationships: is a type of positive regulation of smooth muscle contraction [GO:0045987]; is_a regulation of uterine smooth muscle contraction [GO:0070472]; positively regulates uterine smooth muscle contraction [GO:0070471] Sources: GOC:go_curators